{
  "gene": "UniProtKB:P23416",
  "term_label": "chloride transmembrane transport",
  "gene_symbol": "GLRA2",
  "gene_name": "Glycine receptor subunit alpha-2",
  "term_id": "GO:1902476"
}